{
  "term_id": "UNKNOWN:0001",
  "gene_name": "Transmembrane protein 191B",
  "gene_symbol": "TMEM191B",
  "gene": "UniProtKB:P0C7N4",
  "term_label": "Unknown molecular function"
}